leukocyte mediated cytotoxicity [GO:0001909] (biological process) Regulation: regulated by regulation of leukocyte mediated cytotoxicity [GO:0001910]; negatively regulated by negative regulation of leukocyte mediated cytotoxicity [GO:0001911]; RO_0002213 by positive regulation of leukocyte mediated cytotoxicity [GO:0001912] Relationships: is a type of cell killing [GO:0001906]; is a type of leukocyte mediated immunity [GO:0002443] Definition: The directed killing of a target cell by a leukocyte. References: PMID:11911826 Sources: GOC:add, GO_REF:0000022, ISBN:0781735149 Subtypes: antibody-dependent cellular cytotoxicity [GO:0001788], T cell mediated cytotoxicity [GO:0001913], natural killer cell mediated cytotoxicity [GO:0042267], GO:0070942, GO:0090634 Note: Note that this term and its children describe contact-dependent killing of target cells by lymphocytes and myeloid cells of the immune system. Also known as: immune cell mediated cell death, immune cell mediated cell killing, immune cell mediated cytotoxicity, leucocyte mediated cytotoxicity